amylosucrase activity [GO:0047669] (molecular function) Also known as: sucrose-1,4-alpha-glucan glucosyltransferase activity, sucrose-glucan glucosyltransferase activity, sucrose:1,4-alpha-D-glucan 4-alpha-D-glucosyltransferase activity Sources: EC:2.4.1.4, MetaCyc:AMYLOSUCRASE-RXN Relationships: is a type of hexosyltransferase activity [GO:0016758] Definition: Catalysis of the reaction: sucrose + 1,4-alpha-D-glucosyl(n) = D-fructose + 1,4-alpha-D-glucosyl(n+1).